{
  "gene_symbol": "LNX1",
  "term_label": "ubiquitin-protein transferase activity",
  "term_id": "GO:0004842",
  "gene": "UniProtKB:Q8TBB1",
  "gene_name": "E3 ubiquitin-protein ligase LNX"
}